{
  "gene_symbol": "CENPS",
  "gene": "UniProtKB:Q8N2Z9",
  "term_id": "GO:0031297",
  "gene_name": "Centromere protein S",
  "term_label": "replication fork processing"
}